spindle organization [GO:0007051] (biological process) Sources: GOC:go_curators, GOC:mah Regulation: regulated by GO:0090224 Relationships: is a type of microtubule cytoskeleton organization [GO:0000226]; is a type of cell cycle process [GO:0022402] Definition: A process that is carried out at the cellular level which results in the assembly, arrangement of constituent parts, or disassembly of the spindle, the array of microtubules and associated molecules that forms between opposite poles of a eukaryotic cell during DNA segregation and serves to move the duplicated chromosomes apart. Subtypes: GO:0000212, mitotic spindle organization [GO:0007052], astral microtubule organization [GO:0030953], GO:0051225, spindle disassembly [GO:0051230] Also known as: spindle organisation, spindle organization and biogenesis, spindle stabilization